{
  "gene": "UniProtKB:Q6BDI9",
  "term_id": "GO:0033572",
  "gene_name": "Rab15 effector protein",
  "term_label": "transferrin transport",
  "gene_symbol": "REP15"
}